{
  "term_id": "GO:0004806",
  "term_label": "triacylglycerol lipase activity",
  "gene_symbol": "DAGLB",
  "gene": "UniProtKB:Q8NCG7",
  "gene_name": "Diacylglycerol lipase-beta"
}